{
  "gene_name": "Serine incorporator 5",
  "gene_symbol": "SERINC5",
  "term_label": "membrane",
  "gene": "UniProtKB:Q86VE9",
  "term_id": "GO:0016020"
}